{
  "term_label": "Unknown biological process",
  "gene_symbol": "TRIM33",
  "term_id": "UNKNOWN:0002",
  "gene": "UniProtKB:Q9UPN9",
  "gene_name": "E3 ubiquitin-protein ligase TRIM33"
}